{
  "gene": "UniProtKB:Q9UL46",
  "term_label": "nucleoplasm",
  "gene_symbol": "PSME2",
  "term_id": "GO:0005654",
  "gene_name": "Proteasome activator complex subunit 2"
}